microtubule plus-end [GO:0035371] (cellular component) Subtypes: GO:1904511 Also known as: growing microtubule plus end, microtubule plus end References: PMID:12700769, PMID:16643273 Sources: GOC:bf, GOC:lb Definition: The growing (plus) end of a microtubule. In vitro, microtubules polymerize more quickly at the plus end than at the minus end. In vivo, microtubule growth occurs only at the plus end, and the plus end switches between periods of growth and shortening, a behavior known as dynamic instability. Relationships: is_a GO:1990752